{
  "gene_name": "Heat shock protein HSP 90-alpha",
  "gene": "UniProtKB:P07900",
  "term_label": "protein folding",
  "term_id": "GO:0006457",
  "gene_symbol": "HSP90AA1"
}